nucleoside transmembrane transport [GO:1901642] (biological process) Subtypes: purine nucleoside transmembrane transport [GO:0015860], uridine transmembrane transport [GO:0015862], GO:0160287, nucleoside import across plasma membrane [GO:0180015] Relationships: is_a nucleoside transport [GO:0015858]; is a type of transmembrane transport [GO:0055085] Sources: GOC:TermGenie, GOC:pr Note: Note that this term is not intended for use in annotating lateral movement within membranes. Also known as: nucleoside membrane transport Definition: The directed movement of nucleoside across a membrane.